type I site-specific deoxyribonuclease activity [GO:0009035] (MF) Definition: Catalysis of the endonucleolytic cleavage of DNA to give random double-stranded fragments with terminal 5' or 3' protrusions, driven by ATP hydrolysis. Cleavage is dependent on the presence in the DNA of a specific recognition site. Cleavage may occur hundreds or thousands of base pairs away from the recognition site due to translocation of DNA. Relationships: is a type of DNA translocase activity [GO:0015616]; is a type of restriction endodeoxyribonuclease activity [GO:0015666]; is a type of DNA endonuclease activity, producing 5'-phosphomonoesters [GO:0016888] References: PMID:15300241, PMID:15788748 Also known as: type I restriction enzyme activity, ATP-dependent DNase activity, adenosine triphosphate-dependent deoxyribonuclease activity, deoxyribonuclease (ATP- and S-adenosyl-L-methionine-dependent), deoxyribonuclease (adenosine triphosphate-hydrolyzing)